{
  "gene_symbol": "DYNLT2",
  "term_label": "cytoplasm",
  "gene_name": "Dynein light chain Tctex-type protein 2",
  "gene": "UniProtKB:Q8IZS6",
  "term_id": "GO:0005737"
}